{
  "gene_symbol": "SDHAF2",
  "term_label": "Unknown molecular function",
  "term_id": "UNKNOWN:0001",
  "gene": "UniProtKB:Q9NX18",
  "gene_name": "Succinate dehydrogenase assembly factor 2, mitochondrial"
}